micropexophagy [GO:0000426] (biological process) References: PMID:12914914, PMID:15350980, PMID:16973210 Sources: GOC:autophagy, GOC:pad Note: Note that this term is not a child of pexophagy because the community usually uses the latter to refer to the macroautohagy process. Relationships: is a type of microautophagy [GO:0016237]; is a type of GO:0030242 Definition: Degradation of a peroxisome by microautophagy.